{
  "term_id": "GO:0043218",
  "gene_symbol": "MBP",
  "gene_name": "Myelin basic protein",
  "term_label": "compact myelin",
  "gene": "UniProtKB:P02686"
}